{
  "gene": "UniProtKB:P14679",
  "term_id": "GO:0004503",
  "gene_name": "Tyrosinase",
  "term_label": "tyrosinase activity",
  "gene_symbol": "TYR"
}